{
  "gene_name": "NHS-like protein 1",
  "term_id": "UNKNOWN:0001",
  "gene_symbol": "NHSL1",
  "gene": "UniProtKB:Q5SYE7",
  "term_label": "Unknown molecular function"
}